negative regulation of synaptic vesicle priming [GO:0010809] (biological process) References: PMID:15489511 Sources: GOC:dph, GOC:kmvs, GOC:tb Definition: Any process that decreases the frequency, rate or extent of synaptic vesicle priming. Synaptic vesicle priming is the formation of SNARE-containing complexes, bringing synaptic vesicle membrane and plasma membranes into close proximity and thereby facilitating membrane fusion. Relationships: is a type of regulation of synaptic vesicle priming [GO:0010807]; is a type of negative regulation of protein-containing complex assembly [GO:0031333]; is a type of negative regulation of synaptic vesicle exocytosis [GO:2000301]; negatively regulates synaptic vesicle priming [GO:0016082]